positive regulation of cellular respiration [GO:1901857] (biological process) References: PMID:23150719 Sources: GOC:TermGenie, GOC:yaf Relationships: is a type of positive regulation of metabolic process [GO:0009893]; is a type of regulation of cellular respiration [GO:0043457]; positively regulates cellular respiration [GO:0045333] Also known as: activation of respiration, positive regulation of respiration, up regulation of respiration, up-regulation of respiration, upregulation of respiration, activation of oxidative metabolic process, activation of oxidative metabolism, positive regulation of oxidative metabolic process, positive regulation of oxidative metabolism, up regulation of cellular respiration, up regulation of oxidative metabolic process, up regulation of oxidative metabolism, up-regulation of cellular respiration, up-regulation of oxidative metabolic process, up-regulation of oxidative metabolism, upregulation of cellular respiration, upregulation of oxidative metabolic process, upregulation of oxidative metabolism, activation of cellular respiration Definition: Any process that activates or increases the frequency, rate or extent of cellular respiration. Subtypes: positive regulation of methane biosynthetic process from dimethylamine [GO:1900320], positive regulation of methane biosynthetic process from trimethylamine [GO:1900332], positive regulation of methane biosynthetic process from 3-(methylthio)propionic acid [GO:1900335], positive regulation of methane biosynthetic process from carbon monoxide [GO:1900338], positive regulation of methane biosynthetic process from formic acid [GO:1900341], GO:1900344, positive regulation of methane biosynthetic process from methanethiol [GO:1900347], positive regulation of methane biosynthetic process from methylamine [GO:1900350], positive regulation of mitochondrial electron transport, NADH to ubiquinone [GO:1902958], positive regulation of oxidative phosphorylation [GO:1903862]